{
  "gene_symbol": "GIGYF2",
  "gene_name": "GRB10-interacting GYF protein 2",
  "gene": "UniProtKB:Q6Y7W6",
  "term_id": "GO:0031982",
  "term_label": "vesicle"
}